{
  "gene_name": "Inositol-trisphosphate 3-kinase C",
  "term_id": "GO:0005737",
  "term_label": "cytoplasm",
  "gene": "UniProtKB:Q96DU7",
  "gene_symbol": "ITPKC"
}